negative regulation of inhibitory synapse assembly [GO:1905703] (BP) Also known as: down regulation of inhibitory synapse assembly, down regulation of inhibitory synapse formation, down-regulation of inhibitory synapse assembly, down-regulation of inhibitory synapse formation, downregulation of inhibitory synapse assembly, downregulation of inhibitory synapse formation, negative regulation of inhibitory synapse formation, inhibition of inhibitory synapse assembly, inhibition of inhibitory synapse formation Relationships: is a type of negative regulation of synapse assembly [GO:0051964]; is a type of regulation of inhibitory synapse assembly [GO:1905702]; negatively regulates inhibitory synapse assembly [GO:1904862] Definition: Any process that stops, prevents or reduces the frequency, rate or extent of inhibitory synapse assembly. References: PMID:27779093 Sources: GOC:TermGenie, GO_REF:0000058